{
  "term_label": "Unknown cellular component",
  "term_id": "UNKNOWN:0003",
  "gene": "UniProtKB:P15954",
  "gene_symbol": "COX7C",
  "gene_name": "Cytochrome c oxidase subunit 7C, mitochondrial"
}